{
  "gene_name": "Mitochondrial brown fat uncoupling protein 1",
  "gene": "UniProtKB:P25874",
  "term_label": "proton transmembrane transporter activity",
  "term_id": "GO:0015078",
  "gene_symbol": "UCP1"
}